{
  "term_label": "transmembrane signaling receptor activity",
  "gene_name": "Limb region 1 protein homolog",
  "term_id": "GO:0004888",
  "gene_symbol": "LMBR1",
  "gene": "UniProtKB:Q8WVP7"
}